aortic valve morphogenesis [GO:0003180] (biological process) Relationships: is_a heart valve morphogenesis [GO:0003179]; is part of aortic valve development [GO:0003176] Sources: GOC:mtg_heart Definition: The process in which the structure of the aortic valve is generated and organized.